3' transitive RNA interference [GO:1990515] (biological process) Definition: An RNA interference where the silencing signal spreads 3' along the target mRNA, outside of the initial target sequence. Typically involves the formation of secondary siRNAs formed when the initial mRNA target sequence functions as a template for 5' to 3' synthesis of new dsRNA. References: PMID:24369430 Sources: GOC:pf Relationships: is_a GO:0036453